{
  "term_id": "GO:1903278",
  "gene_name": "FXYD domain-containing ion transport regulator 3",
  "gene_symbol": "FXYD3",
  "gene": "UniProtKB:Q14802",
  "term_label": "positive regulation of sodium ion export across plasma membrane"
}